{
  "term_label": "Unknown biological process",
  "gene_symbol": "OR6C4",
  "gene": "UniProtKB:Q8NGE1",
  "gene_name": "Olfactory receptor 6C4",
  "term_id": "UNKNOWN:0002"
}